{
  "gene_symbol": "LACTB",
  "term_id": "GO:0006508",
  "gene_name": "Serine beta-lactamase-like protein LACTB, mitochondrial",
  "gene": "UniProtKB:P83111",
  "term_label": "proteolysis"
}